{
  "gene_name": "Serine dehydratase-like",
  "gene": "UniProtKB:Q96GA7",
  "term_id": "GO:0004794",
  "term_label": "threonine deaminase activity",
  "gene_symbol": "SDSL"
}